micropinosome [GO:0044353] (cellular component) Definition: A membrane-bounded, uncoated intracellular vesicle formed by the process of micropinocytosis. References: PMID:14731589, PMID:14732047 Relationships: is a type of GO:0044352